{
  "term_id": "UNKNOWN:0001",
  "gene": "UniProtKB:Q96NT3",
  "term_label": "Unknown molecular function",
  "gene_symbol": "GUCD1",
  "gene_name": "Protein GUCD1"
}